{
  "term_label": "D-glutamate cyclase activity",
  "gene_symbol": "DGLUCY",
  "term_id": "GO:0047820",
  "gene": "UniProtKB:Q7Z3D6",
  "gene_name": "D-glutamate cyclase, mitochondrial"
}